regulation of systemic arterial blood pressure by baroreceptor feedback [GO:0003025] (biological process) Relationships: is a type of nervous system process involved in regulation of systemic arterial blood pressure [GO:0001976] Also known as: baroreceptor regulation of systemic arterial blood pressure Definition: The neural regulation of blood pressure in which baroreceptors sense the amount of stretch occurring in vessels and respond to the input via central nervous system control. Sources: GOC:dph, GOC:mtg_cardio, GOC:tb